{
  "gene_symbol": "GRIN2A",
  "gene_name": "Glutamate receptor ionotropic, NMDA 2A",
  "gene": "UniProtKB:Q12879",
  "term_id": "GO:0098839",
  "term_label": "postsynaptic density membrane"
}